{
  "gene_symbol": "SCGB1C1",
  "term_label": "Unknown cellular component",
  "gene": "UniProtKB:Q8TD33",
  "gene_name": "Secretoglobin family 1C member 1",
  "term_id": "UNKNOWN:0003"
}